{
  "gene_name": "Guanidinoacetate N-methyltransferase",
  "gene_symbol": "GAMT",
  "term_label": "nucleus",
  "gene": "UniProtKB:Q14353",
  "term_id": "GO:0005634"
}